{
  "gene_name": "WD repeat-containing protein WRAP73",
  "gene_symbol": "WRAP73",
  "term_label": "MWP complex",
  "term_id": "GO:1990811",
  "gene": "UniProtKB:Q9P2S5"
}